{
  "term_label": "Unknown cellular component",
  "gene": "UniProtKB:Q6UW10",
  "gene_name": "Surfactant-associated protein 2",
  "term_id": "UNKNOWN:0003",
  "gene_symbol": "SFTA2"
}